{
  "gene_symbol": "FAM86B1",
  "term_id": "UNKNOWN:0002",
  "gene_name": "Putative protein N-methyltransferase FAM86B1",
  "term_label": "Unknown biological process",
  "gene": "UniProtKB:Q8N7N1"
}